{
  "gene": "UniProtKB:Q8IWV8",
  "gene_symbol": "UBR2",
  "term_label": "protein ubiquitination",
  "gene_name": "E3 ubiquitin-protein ligase UBR2",
  "term_id": "GO:0016567"
}